{
  "gene": "UniProtKB:A8MUN3",
  "gene_name": "Putative uncharacterized protein ENSP00000381830",
  "gene_symbol": "A8MUN3",
  "term_id": "UNKNOWN:0003",
  "term_label": "Unknown cellular component"
}